{
  "gene": "UniProtKB:Q9NYC9",
  "term_id": "GO:0045505",
  "gene_name": "Dynein axonemal heavy chain 9",
  "gene_symbol": "DNAH9",
  "term_label": "dynein intermediate chain binding"
}